flap endonuclease activity [GO:0048256] (MF) Definition: Catalysis of the cleavage of a flap structure in DNA, but not other DNA structures; processes the ends of Okazaki fragments in lagging strand DNA synthesis. Relationships: is a type of DNA endonuclease activity [GO:0004520]; is a type of hydrolase activity, acting on ester bonds [GO:0016788] Subtypes: GO:0017108, 3'-flap endonuclease activity [GO:0048257] Sources: GOC:jid